{
  "gene_symbol": "TRIM45",
  "term_label": "ubiquitin protein ligase activity",
  "gene_name": "E3 ubiquitin-protein ligase TRIM45",
  "term_id": "GO:0061630",
  "gene": "UniProtKB:Q9H8W5"
}